{
  "gene_symbol": "TMEM107",
  "gene_name": "Transmembrane protein 107",
  "term_label": "protein localization to ciliary transition zone",
  "gene": "UniProtKB:Q6UX40",
  "term_id": "GO:1904491"
}